chitin-based embryonic cuticle biosynthetic process [GO:0008362] (biological process) Also known as: embryonic cuticle anabolism, embryonic cuticle biosynthetic process, embryonic cuticle formation, embryonic cuticle synthesis Relationships: is a type of chitin-based cuticle development [GO:0040003] References: PMID:12019232 Sources: GOC:bf, GOC:mtg_sensu Definition: Synthesis, including the chemical reactions and pathways resulting in the formation of chitin and other components, and deposition of a chitin-based embryonic cuticle by the underlying epidermal epithelium. This tough, waterproof cuticle layer is essential to provide structural integrity of the larval body. An example of this is found in Drosophila melanogaster.